{
  "gene": "UniProtKB:P14415",
  "gene_symbol": "ATP1B2",
  "gene_name": "Sodium_potassium-transporting ATPase subunit beta-2",
  "term_label": "sodium:potassium-exchanging ATPase complex",
  "term_id": "GO:0005890"
}